protein localization to equatorial microtubule organizing center [GO:1904759] (biological process) Relationships: is a type of protein localization to cell division site [GO:0072741]; is a type of protein localization to microtubule organizing center [GO:1905508] Also known as: protein localisation in equatorial microtubule organizing center, protein localisation to equatorial microtubule organizing center, protein localization in equatorial microtubule organizing center, protein localization to eMTOC Definition: A process in which a protein is transported to, or maintained in, a location within an equatorial microtubule organizing center. References: PMID:16611237 Sources: GOC:TermGenie, GO_REF:0000087